{
  "gene_symbol": "RC3H2",
  "term_label": "nuclear-transcribed mRNA catabolic process, deadenylation-dependent decay",
  "term_id": "GO:0000288",
  "gene": "UniProtKB:Q9HBD1",
  "gene_name": "Roquin-2"
}